{
  "gene_symbol": "ACO1",
  "term_id": "GO:0051539",
  "term_label": "4 iron, 4 sulfur cluster binding",
  "gene_name": "Cytoplasmic aconitate hydratase",
  "gene": "UniProtKB:P21399"
}